{
  "term_id": "GO:0045892",
  "gene": "UniProtKB:Q13263",
  "gene_name": "Transcription intermediary factor 1-beta",
  "gene_symbol": "TRIM28",
  "term_label": "negative regulation of DNA-templated transcription"
}